{
  "gene_name": "Rho-related GTP-binding protein RhoU",
  "term_id": "GO:0030010",
  "term_label": "establishment of cell polarity",
  "gene": "UniProtKB:Q7L0Q8",
  "gene_symbol": "RHOU"
}